{
  "gene": "UniProtKB:O43610",
  "gene_name": "Protein sprouty homolog 3",
  "term_label": "protein kinase inhibitor activity",
  "term_id": "GO:0004860",
  "gene_symbol": "SPRY3"
}